{
  "term_id": "GO:0005643",
  "gene_name": "Aladin",
  "gene": "UniProtKB:Q9NRG9",
  "gene_symbol": "AAAS",
  "term_label": "nuclear pore"
}